{
  "gene_name": "Trafficking protein particle complex subunit 10",
  "gene_symbol": "TRAPPC10",
  "term_id": "GO:0005085",
  "term_label": "guanyl-nucleotide exchange factor activity",
  "gene": "UniProtKB:P48553"
}